{
  "gene_name": "Alpha-protein kinase 1",
  "gene_symbol": "ALPK1",
  "gene": "UniProtKB:Q96QP1",
  "term_label": "cytoplasmic pattern recognition receptor signaling pathway",
  "term_id": "GO:0002753"
}